{
  "term_id": "GO:0005770",
  "gene": "UniProtKB:Q8N3P4",
  "gene_symbol": "VPS8",
  "term_label": "late endosome",
  "gene_name": "Vacuolar protein sorting-associated protein 8 homolog"
}